{
  "gene_name": "Heat shock-related 70 kDa protein 2",
  "gene_symbol": "HSPA2",
  "term_id": "GO:0031072",
  "term_label": "heat shock protein binding",
  "gene": "UniProtKB:P54652"
}